{
  "gene": "UniProtKB:Q9NQW7",
  "gene_symbol": "XPNPEP1",
  "term_id": "UNKNOWN:0001",
  "term_label": "Unknown molecular function",
  "gene_name": "Xaa-Pro aminopeptidase 1"
}